{
  "term_id": "GO:0012505",
  "term_label": "endomembrane system",
  "gene": "UniProtKB:Q92604",
  "gene_name": "Acyl-CoA:lysophosphatidylglycerol acyltransferase 1",
  "gene_symbol": "LPGAT1"
}